(RS)-1-benzyl-1,2,3,4-tetrahydroisoquinoline N-methyltransferase activity [GO:0030776] (molecular function) Definition: Catalysis of the reaction: S-adenosyl-L-methionine + (RS)-1-benzyl-1,2,3,4-tetrahydroisoquinoline = S-adenosyl-L-homocysteine + N-methyl-(RS)-1-benzyl-1,2,3,4-tetrahydroisoquinoline. Sources: EC:2.1.1.115 Also known as: (RS)-tetrahydrobenzylisoquinoline N-methyltransferase activity, S-adenosyl-L-methionine:(RS)-1-benzyl-1,2,3,4-tetrahydroisoquinoline N-methyltransferase activity, norreticuline N-methyltransferase activity Relationships: is a type of S-adenosylmethionine-dependent methyltransferase activity [GO:0008757]